{
  "gene_name": "Proline-rich protein 20E",
  "gene": "UniProtKB:P86478",
  "term_label": "Unknown biological process",
  "term_id": "UNKNOWN:0002",
  "gene_symbol": "PRR20E"
}